{
  "gene": "UniProtKB:Q8NDX9",
  "term_label": "Unknown molecular function",
  "term_id": "UNKNOWN:0001",
  "gene_symbol": "LY6G5B",
  "gene_name": "Lymphocyte antigen 6 complex locus protein G5b"
}